{
  "gene": "UniProtKB:P07510",
  "term_label": "acetylcholine receptor activity",
  "gene_name": "Acetylcholine receptor subunit gamma",
  "gene_symbol": "CHRNG",
  "term_id": "GO:0015464"
}